regulation of microlipophagy [GO:0140505] (biological process) Relationships: is a type of regulation of autophagy [GO:0010506]; regulates microlipophagy [GO:0140504] Definition: Any process that modulates the frequency, rate or extent of microlipophagy, the microautophagy-mediated direct internalization of lipid droplets into a lysosome-like vacuole during nutrient depletion. References: PMID:28394250, PMID:29601311